{
  "gene_name": "Olfactory receptor 7G1",
  "term_id": "GO:0004984",
  "gene": "UniProtKB:Q8NGA0",
  "term_label": "olfactory receptor activity",
  "gene_symbol": "OR7G1"
}